{
  "term_label": "serine hydrolase activity",
  "gene_symbol": "NCEH1",
  "term_id": "GO:0017171",
  "gene": "UniProtKB:Q6PIU2",
  "gene_name": "Neutral cholesterol ester hydrolase 1"
}